{
  "gene_name": "E3 ubiquitin-protein ligase RNF169",
  "gene_symbol": "RNF169",
  "term_label": "double-strand break repair",
  "gene": "UniProtKB:Q8NCN4",
  "term_id": "GO:0006302"
}